{
  "term_id": "GO:0051932",
  "term_label": "synaptic transmission, GABAergic",
  "gene_name": "Gamma-aminobutyric acid receptor subunit alpha-3",
  "gene": "UniProtKB:P34903",
  "gene_symbol": "GABRA3"
}